{
  "term_label": "endoplasmic reticulum membrane",
  "gene_name": "Sterol regulatory element-binding protein cleavage-activating protein",
  "gene": "UniProtKB:Q12770",
  "term_id": "GO:0005789",
  "gene_symbol": "SCAP"
}